{
  "term_label": "RNA polymerase II transcription regulator complex",
  "term_id": "GO:0090575",
  "gene_name": "Thyroid hormone receptor alpha",
  "gene_symbol": "THRA",
  "gene": "UniProtKB:P10827"
}